{
  "term_label": "rDNA heterochromatin",
  "term_id": "GO:0033553",
  "gene": "UniProtKB:O43159",
  "gene_symbol": "RRP8",
  "gene_name": "Ribosomal RNA-processing protein 8"
}